{
  "gene_name": "Protein Aster-C",
  "term_label": "endoplasmic reticulum membrane",
  "term_id": "GO:0005789",
  "gene_symbol": "GRAMD1C",
  "gene": "UniProtKB:Q8IYS0"
}